{
  "gene": "UniProtKB:P49711",
  "term_id": "UNKNOWN:0003",
  "term_label": "Unknown cellular component",
  "gene_name": "Transcriptional repressor CTCF",
  "gene_symbol": "CTCF"
}